regulation of renal water transport [GO:2001151] (biological process) Sources: GOC:obol Relationships: is a type of GO:0050878; is a type of GO:0051049; is a type of regulation of renal system process [GO:0098801]; regulates renal water transport [GO:0003097] Definition: Any process that modulates the frequency, rate or extent of renal water transport. Subtypes: GO:2001152, positive regulation of renal water transport [GO:2001153]